{
  "term_id": "UNKNOWN:0001",
  "gene": "UniProtKB:O00559",
  "gene_symbol": "EBAG9",
  "gene_name": "Receptor-binding cancer antigen expressed on SiSo cells",
  "term_label": "Unknown molecular function"
}